{
  "gene_symbol": "PIP5KL1",
  "gene_name": "Phosphatidylinositol 4-phosphate 5-kinase-like protein 1",
  "gene": "UniProtKB:Q5T9C9",
  "term_id": "GO:0005886",
  "term_label": "plasma membrane"
}